{
  "term_id": "GO:0006612",
  "gene_symbol": "VPS37D",
  "term_label": "protein targeting to membrane",
  "gene": "UniProtKB:Q86XT2",
  "gene_name": "Vacuolar protein sorting-associated protein 37D"
}